{
  "gene_symbol": "TTC28",
  "term_id": "UNKNOWN:0003",
  "gene_name": "Tetratricopeptide repeat protein 28",
  "term_label": "Unknown cellular component",
  "gene": "UniProtKB:Q96AY4"
}